{
  "term_id": "GO:0098839",
  "gene": "UniProtKB:P62955",
  "term_label": "postsynaptic density membrane",
  "gene_name": "Voltage-dependent calcium channel gamma-7 subunit",
  "gene_symbol": "CACNG7"
}